{
  "term_id": "GO:0098839",
  "gene": "UniProtKB:P42261",
  "gene_name": "Glutamate receptor 1",
  "term_label": "postsynaptic density membrane",
  "gene_symbol": "GRIA1"
}